{
  "gene_name": "Testis-expressed protein 13B",
  "gene": "UniProtKB:Q9BXU2",
  "gene_symbol": "TEX13B",
  "term_id": "UNKNOWN:0003",
  "term_label": "Unknown cellular component"
}